cellular response to interleukin-3 [GO:0036016] (biological process) Definition: Any process that results in a change in state or activity of a cell (in terms of movement, secretion, enzyme production, gene expression, etc.) as a result of an interleukin-3 stimulus. Sources: GOC:yaf Also known as: cellular response to IL-3 Relationships: is_a response to interleukin-3 [GO:0036015]; is a type of cellular response to cytokine stimulus [GO:0071345]